{
  "term_id": "GO:0000076",
  "gene_name": "Cell cycle checkpoint control protein RAD9B",
  "term_label": "DNA replication checkpoint signaling",
  "gene_symbol": "RAD9B",
  "gene": "UniProtKB:Q6WBX8"
}